{
  "gene": "UniProtKB:P24588",
  "gene_name": "A-kinase anchor protein 5",
  "term_id": "GO:0050811",
  "gene_symbol": "AKAP5",
  "term_label": "GABA receptor binding"
}